excinuclease ABC activity [GO:0009381] (molecular function) Relationships: is a type of DNA endonuclease activity [GO:0004520]; is a type of GO:0016788 Definition: Catalysis of the hydrolysis of ester linkages within deoxyribonucleic acid at sites flanking regions of damaged DNA to which the Uvr ABC excinuclease complexes bind. References: PMID:15192705 Sources: GOC:mah